{
  "gene_name": "Keratin, type I cytoskeletal 26",
  "term_id": "GO:0002009",
  "gene": "UniProtKB:Q7Z3Y9",
  "term_label": "morphogenesis of an epithelium",
  "gene_symbol": "KRT26"
}